{
  "term_label": "angiogenesis",
  "gene": "UniProtKB:Q9H6I2",
  "gene_symbol": "SOX17",
  "term_id": "GO:0001525",
  "gene_name": "Transcription factor SOX-17"
}